{
  "gene_symbol": "KRT13",
  "term_id": "GO:0002009",
  "gene_name": "Keratin, type I cytoskeletal 13",
  "term_label": "morphogenesis of an epithelium",
  "gene": "UniProtKB:P13646"
}